DNA topoisomerase activity [GO:0003916] (molecular function) References: PMID:8811192 Sources: GOC:mah Definition: Catalysis of the transient cleavage and passage of individual DNA strands or double helices through one another, resulting a topological transformation in double-stranded DNA. Relationships: is a type of nucleic acid conformation isomerase activity [GO:0120545]; is a type of catalytic activity, acting on DNA [GO:0140097]; has part DNA binding [GO:0003677] Subtypes: DNA topoisomerase type I (single strand cut, ATP-independent) activity [GO:0003917], DNA topoisomerase type II (double strand cut, ATP-hydrolyzing) activity [GO:0003918], GO:0160097